isoguanine deaminase activity [GO:0035888] (molecular function) Definition: Catalysis of the reaction: H+ + H2O + isoguanine = NH4+ + xanthine. References: PMID:21604715 Sources: RHEA:47720 Also known as: 2-hydroxyadenine deaminase activity, 2-oxoadenine deaminase activity Relationships: is a type of hydrolase activity, acting on carbon-nitrogen (but not peptide) bonds, in cyclic amidines [GO:0016814]; is a type of deaminase activity [GO:0019239]